{
  "gene_name": "Homeobox protein Hox-C8",
  "term_id": "GO:0000981",
  "gene_symbol": "HOXC8",
  "term_label": "DNA-binding transcription factor activity, RNA polymerase II-specific",
  "gene": "UniProtKB:P31273"
}